{
  "gene_name": "Osteocrin",
  "gene": "UniProtKB:P61366",
  "gene_symbol": "OSTN",
  "term_label": "signaling receptor binding",
  "term_id": "GO:0005102"
}